{
  "gene_symbol": "PIWIL2",
  "gene": "UniProtKB:Q8TC59",
  "term_id": "GO:0004521",
  "term_label": "RNA endonuclease activity",
  "gene_name": "Piwi-like protein 2"
}